Grb2-EGFR complex [GO:0070436] (cellular component) Also known as: Grb2-Egfr complex, EGF stimulated Relationships: is a type of plasma membrane protein complex [GO:0098797] Definition: A protein complex that contains the epidermal growth factor receptor (EGFR) and Grb2, and is involved in linking EGFR activation to the p21-Ras pathway. References: PMID:7798267 Sources: GOC:mah